cellular response to gibberellin stimulus [GO:0071370] (biological process) Also known as: cellular response to gibberellic acid stimulus Relationships: is a type of response to gibberellin [GO:0009739]; is a type of cellular response to hormone stimulus [GO:0032870]; is a type of GO:0071396; is a type of cellular response to oxygen-containing compound [GO:1901701] Sources: GOC:mah Definition: Any process that results in a change in state or activity of a cell (in terms of movement, secretion, enzyme production, gene expression, etc.) as a result of a gibberellin stimulus.